{
  "term_label": "tRNA-specific adenosine deaminase activity",
  "gene": "UniProtKB:Q9BUB4",
  "term_id": "GO:0008251",
  "gene_name": "tRNA-specific adenosine deaminase 1",
  "gene_symbol": "ADAT1"
}